{
  "term_label": "immune response",
  "gene": "UniProtKB:P25025",
  "gene_name": "C-X-C chemokine receptor type 2",
  "term_id": "GO:0006955",
  "gene_symbol": "CXCR2"
}